{
  "gene_symbol": "AMY2A",
  "term_label": "carbohydrate metabolic process",
  "gene_name": "Pancreatic alpha-amylase",
  "term_id": "GO:0005975",
  "gene": "UniProtKB:P04746"
}